double-stranded DNA helicase activity [GO:0036121] (molecular function) Relationships: is a type of GO:0003678 Definition: Catalysis of the reaction: ATP + H2O = ADP + phosphate, in the presence of double-stranded DNA; drives the unwinding of a DNA helix. Sources: GOC:kmv Also known as: double-stranded DNA-dependent ATP-dependent DNA helicase activity, double-stranded DNA-dependent ATPase activity, dsDNA-dependent ATP-dependent DNA helicase activity, dsDNA-dependent ATPase activity